{
  "gene": "UniProtKB:Q8IUE6",
  "term_label": "nucleus",
  "gene_symbol": "H2AC21",
  "term_id": "GO:0005634",
  "gene_name": "Histone H2A type 2-B"
}